{
  "gene_name": "Cis-aconitate decarboxylase",
  "gene": "UniProtKB:A6NK06",
  "term_id": "GO:0045824",
  "gene_symbol": "ACOD1",
  "term_label": "negative regulation of innate immune response"
}